{
  "gene_name": "Mucin-2",
  "term_id": "UNKNOWN:0001",
  "gene_symbol": "MUC2",
  "term_label": "Unknown molecular function",
  "gene": "UniProtKB:Q02817"
}